{
  "gene": "UniProtKB:Q8NA57",
  "term_label": "poly(A)+ mRNA export from nucleus",
  "gene_name": "Uncharacterized protein C12orf50",
  "gene_symbol": "C12orf50",
  "term_id": "GO:0016973"
}